{
  "gene": "UniProtKB:Q96S65",
  "gene_symbol": "CSRNP1",
  "term_label": "DNA-binding transcription factor activity, RNA polymerase II-specific",
  "term_id": "GO:0000981",
  "gene_name": "Cysteine_serine-rich nuclear protein 1"
}